{
  "gene": "UniProtKB:Q8NB14",
  "gene_symbol": "USP38",
  "term_label": "nucleus",
  "gene_name": "Ubiquitin carboxyl-terminal hydrolase 38",
  "term_id": "GO:0005634"
}